{
  "gene_name": "Immunoglobulin lambda constant 7",
  "term_id": "GO:0003823",
  "gene": "UniProtKB:A0M8Q6",
  "term_label": "antigen binding",
  "gene_symbol": "IGLC7"
}